blue light photoreceptor activity [GO:0009882] (MF) Definition: The function of absorbing and responding to electromagnetic radiation with a wavelength of approximately 400-470nm. The response may involve a change in conformation. Relationships: is a type of photoreceptor activity [GO:0009881]; is part of blue light signaling pathway [GO:0009785] Sources: GOC:tb